{
  "gene": "UniProtKB:Q49AN0",
  "term_label": "FAD binding",
  "gene_symbol": "CRY2",
  "term_id": "GO:0071949",
  "gene_name": "Cryptochrome-2"
}